{
  "gene": "UniProtKB:Q96LZ2",
  "gene_symbol": "MAGEB10",
  "term_id": "UNKNOWN:0001",
  "gene_name": "Melanoma-associated antigen B10",
  "term_label": "Unknown molecular function"
}